regulation of cellulose catabolic process [GO:2000997] (biological process) Sources: GOC:mengo_curators Subtypes: GO:2000998, positive regulation of cellulose catabolic process [GO:2000999] Definition: Any process that modulates the frequency, rate or extent of cellulose catabolic process. Also known as: regulation of cellulose breakdown, regulation of cellulose catabolism, regulation of cellulose degradation Relationships: is_a regulation of beta-glucan metabolic process [GO:0032950]; is a type of regulation of carbohydrate catabolic process [GO:0043470]; regulates cellulose catabolic process [GO:0030245]